negative regulation of post-embryonic development [GO:0048581] (biological process) Also known as: down regulation of post-embryonic development, down-regulation of post-embryonic development, downregulation of post-embryonic development, inhibition of post-embryonic development Definition: Any process that stops, prevents, or reduces the frequency, rate or extent of post-embryonic development. Post-embryonic development is defined as the process whose specific outcome is the progression of the organism over time, from the completion of embryonic development to the mature structure. Relationships: is a type of regulation of post-embryonic development [GO:0048580]; is a type of negative regulation of developmental process [GO:0051093]; is a type of negative regulation of multicellular organismal process [GO:0051241]; negatively regulates post-embryonic development [GO:0009791] Sources: GOC:jid Subtypes: negative regulation of flower development [GO:0009910], negative regulation of photomorphogenesis [GO:0010100], GO:0010187, negative regulation of short-day photoperiodism, flowering [GO:0048577], negative regulation of long-day photoperiodism, flowering [GO:0048579], negative regulation of nematode larval development [GO:0061064], negative regulation of pupariation [GO:0106024], negative regulation of thermomorphogenesis [GO:0140921], negative regulation of lateral root development [GO:1901332], negative regulation of stomatal complex development [GO:2000122]